6,7-dimethyl-8-ribityllumazine synthase activity [GO:0000906] (molecular function) References: PMID:7559556 Relationships: is a type of transferase activity, transferring alkyl or aryl (other than methyl) groups [GO:0016765] Definition: Catalysis of the reaction: 3,4-dihydroxy-2-butanone-4-phosphate + 5-amino-6-ribitylamino-2,4(1H,3H)-pyrimidinedione = 6,7-dimethyl-8-ribityllumazine + phosphate. Also known as: lumazine synthase activity